{
  "gene": "UniProtKB:Q8IXS2",
  "term_label": "axonemal dynein complex assembly",
  "term_id": "GO:0070286",
  "gene_symbol": "CCDC65",
  "gene_name": "Dynein regulatory complex subunit 2"
}